quercetin biosynthetic process [GO:1901734] (biological process) Definition: The chemical reactions and pathways resulting in the formation of quercetin. Relationships: is a type of flavone biosynthetic process [GO:0051553] Also known as: quercetin anabolism, quercetin biosynthesis, quercetin formation, quercetin synthesis Sources: GOC:TermGenie, GOC:yaf, UniPathway:UPA00724